{
  "gene": "UniProtKB:Q96PS8",
  "term_id": "GO:0006833",
  "gene_name": "Aquaporin-10",
  "gene_symbol": "AQP10",
  "term_label": "water transport"
}